{
  "gene_name": "HMG domain-containing protein 4",
  "gene_symbol": "HMGXB4",
  "term_id": "UNKNOWN:0003",
  "term_label": "Unknown cellular component",
  "gene": "UniProtKB:Q9UGU5"
}